(S)-methylmalonyl-CoA hydrolase activity [GO:0047511] (molecular function) Also known as: D-methylmalonyl-coenzyme A hydrolase activity Sources: EC:3.1.2.17, RHEA:17345 Definition: Catalysis of the reaction: (S)-methylmalonyl-CoA + H2O = CoA + H+ + methylmalonate. Relationships: is a type of GO:0016289